{
  "term_id": "GO:0005634",
  "term_label": "nucleus",
  "gene_name": "Helicase-like transcription factor",
  "gene_symbol": "HLTF",
  "gene": "UniProtKB:Q14527"
}